{
  "gene_name": "Dihydropyrimidinase-related protein 1",
  "gene_symbol": "CRMP1",
  "gene": "UniProtKB:Q14194",
  "term_label": "Unknown biological process",
  "term_id": "UNKNOWN:0002"
}